{
  "term_id": "GO:0007189",
  "gene_name": "Melanocyte-stimulating hormone receptor",
  "gene": "UniProtKB:Q01726",
  "term_label": "adenylate cyclase-activating G protein-coupled receptor signaling pathway",
  "gene_symbol": "MC1R"
}